Fc receptor mediated inhibitory signaling pathway [GO:0002774] (biological process) Also known as: Fc receptor mediated inhibitory signalling pathway, Fc-receptor mediated inhibitory signaling pathway Sources: GOC:add, ISBN:0781735149 Relationships: is a type of immune response-inhibiting cell surface receptor signaling pathway [GO:0002767] Definition: The series of molecular signals generated as a consequence of the binding of the Fc portion of an immunoglobulin by an Fc receptor capable of inhibiting an immune effector process contributing to an immune response. The Fc portion of an immunoglobulin is its C-terminal constant region.